{
  "gene_symbol": "MELTF",
  "term_id": "GO:0006826",
  "gene_name": "Melanotransferrin",
  "term_label": "iron ion transport",
  "gene": "UniProtKB:P08582"
}